{
  "term_id": "UNKNOWN:0001",
  "gene_symbol": "POLR3C",
  "gene": "UniProtKB:Q9BUI4",
  "term_label": "Unknown molecular function",
  "gene_name": "DNA-directed RNA polymerase III subunit RPC3"
}